protein localization involved in establishment of planar polarity [GO:0090251] (biological process) Definition: Any process in which a protein is transported to, and/or maintained in, a specific location in a cell that contributes to the establishment of planar polarity. Sources: GOC:ascb_2009, GOC:dph, GOC:tb Also known as: protein localisation involved in establishment of planar polarity Relationships: is a type of intracellular protein localization [GO:0008104]; is part of GO:0001736